{
  "gene": "UniProtKB:Q9H7Y0",
  "gene_name": "Divergent protein kinase domain 2B",
  "gene_symbol": "DIPK2B",
  "term_label": "Unknown biological process",
  "term_id": "UNKNOWN:0002"
}